{
  "term_label": "cholesterol efflux",
  "gene_name": "ATP-binding cassette sub-family G member 8",
  "term_id": "GO:0033344",
  "gene_symbol": "ABCG8",
  "gene": "UniProtKB:Q9H221"
}